cellulose catabolic process [GO:0030245] (biological process) Also known as: cellulose breakdown, cellulose catabolism, cellulose degradation Subtypes: GO:0052785, anaerobic cellulose catabolic process [GO:1990488] Regulation: regulated by GO:2000997; negatively regulated by negative regulation of cellulose catabolic process [GO:2000998]; positively regulated by positive regulation of cellulose catabolic process [GO:2000999] Definition: The chemical reactions and pathways resulting in the breakdown of cellulose, a linear beta1-4 glucan of molecular mass 50-400 kDa with the pyranose units in the -4C1 conformation. Sources: GOC:mah, ISBN:0198506732 Relationships: is a type of cellulose metabolic process [GO:0030243]; is a type of beta-glucan catabolic process [GO:0051275]